vitamin A transport [GO:0071938] (biological process) Relationships: is a type of terpenoid transport [GO:0046865]; is a type of vitamin transport [GO:0051180] References: PMID:16011460, PMID:1924551 Sources: GOC:mah Also known as: vitamin A uptake and transport Definition: The directed movement any form of vitamin A into, out of or within a cell, or between cells, by means of some agent such as a transporter or pore. Vitamin A is any of several retinoid derivatives of beta-carotene, primarily retinol, retinal, or retinoic acid. Subtypes: vitamin A import into cell [GO:0071939]